{
  "gene_name": "Male-enhanced antigen 1",
  "term_label": "Unknown molecular function",
  "gene": "UniProtKB:Q16626",
  "term_id": "UNKNOWN:0001",
  "gene_symbol": "MEA1"
}